regulation of myeloid cell apoptotic process [GO:0033032] (biological process) Definition: Any process that modulates the frequency, rate, or extent of myeloid cell apoptotic process. Sources: GOC:add, GOC:mtg_apoptosis Subtypes: GO:0033025, regulation of neutrophil apoptotic process [GO:0033029], GO:0033033, positive regulation of myeloid cell apoptotic process [GO:0033034], GO:1902250, regulation of macrophage apoptotic process [GO:2000109] Relationships: is a type of regulation of apoptotic process [GO:0042981]; RO_0002211 myeloid cell apoptotic process [GO:0033028] Also known as: regulation of myeloid cell apoptosis